{
  "gene_symbol": "ARID5A",
  "term_label": "regulation of transcription by RNA polymerase II",
  "gene_name": "AT-rich interactive domain-containing protein 5A",
  "gene": "UniProtKB:Q03989",
  "term_id": "GO:0006357"
}